{
  "term_id": "GO:0000122",
  "gene_name": "Period circadian protein homolog 3",
  "gene_symbol": "PER3",
  "term_label": "negative regulation of transcription by RNA polymerase II",
  "gene": "UniProtKB:P56645"
}